1,4-dihydroxy-2-naphthoyl-CoA synthase activity [GO:0008935] (molecular function) Also known as: DHNA synthetase activity, O-succinylbenzoyl-CoA 1,4-dihydroxy-2-naphthoate-lyase (cyclizing) activity, dihydroxynaphthoate synthase activity, dihydroxynaphthoic acid synthetase activity, naphthoate synthase activity Sources: RHEA:26562 Relationships: is a type of oxo-acid-lyase activity [GO:0016833] Definition: Catalysis of the reaction: 2-succinylbenzoyl-CoA + H+ = 1,4-dihydroxy-2-naphthoyl-CoA + H2O.